{
  "gene_symbol": "SYNGR1",
  "term_label": "Unknown biological process",
  "gene_name": "Synaptogyrin-1",
  "term_id": "UNKNOWN:0002",
  "gene": "UniProtKB:O43759"
}